{
  "gene_name": "Dynein regulatory complex subunit 2",
  "term_label": "cilium-dependent cell motility",
  "term_id": "GO:0060285",
  "gene": "UniProtKB:Q8IXS2",
  "gene_symbol": "CCDC65"
}